regulation of termination of RNA polymerase II transcription, poly(A)-coupled [GO:2000804] (biological process) Definition: Any process that modulates the frequency, rate or extent of termination of RNA polymerase II transcription, poly(A)-coupled. Relationships: is a type of regulation of termination of RNA polymerase II transcription [GO:1904594]; RO_0002211 GO:0030846 Sources: GOC:obol Also known as: regulation of termination of RNA polymerase II transcription, polyadenylation-coupled, regulation of transcription termination from Pol II promoter, RNA polymerase(A) coupled, regulation of transcription termination from Pol II promoter, poly(A) coupled Subtypes: negative regulation of termination of RNA polymerase II transcription, poly(A)-coupled [GO:2000805], positive regulation of termination of RNA polymerase II transcription, poly(A)-coupled [GO:2000806]